glycolipid biosynthetic process [GO:0009247] (biological process) Definition: The chemical reactions and pathways resulting in the formation of glycolipid, a class of 1,2-di-O-acylglycerols joined at oxygen 3 by a glycosidic linkage to a carbohydrate part (usually a mono-, di- or tri-saccharide). Sources: GOC:go_curators Also known as: glycolipid anabolism, glycolipid biosynthesis, glycolipid formation, glycolipid synthesis Relationships: is a type of glycolipid metabolic process [GO:0006664]; is a type of membrane lipid biosynthetic process [GO:0046467]; is a type of GO:1901137 Subtypes: GPI anchor biosynthetic process [GO:0006506], GO:0006688, GO:0009245, GO:0019347, galactolipid biosynthetic process [GO:0019375], sophorosyloxydocosanoate biosynthetic process [GO:0019435], Kdo2-lipid A biosynthetic process [GO:0036104], 4-amino-4-deoxy-alpha-L-arabinopyranosyl undecaprenyl phosphate biosynthetic process [GO:0036108], GO:0097093, rhamnolipid biosynthesis [GO:0106236], GO:0180047, beta-L-Ara4N-lipid A biosynthetic process [GO:1901760]